negative regulation of collateral sprouting [GO:0048671] (BP) Sources: GOC:dgh, GOC:dph, GOC:jid, GOC:lm Subtypes: negative regulation of collateral sprouting of intact axon in response to injury [GO:0048685], negative regulation of collateral sprouting of injured axon [GO:0048695], GO:0048698 Relationships: is a type of GO:0030308; is a type of GO:0048640; is a type of GO:0048670; is a type of negative regulation of axonogenesis [GO:0050771]; negatively regulates collateral sprouting [GO:0048668] Also known as: down regulation of collateral sprouting, down-regulation of collateral sprouting, downregulation of collateral sprouting, inhibition of collateral sprouting Definition: Any process that stops, prevents, or reduces the frequency, rate or extent of collateral sprouting.